{
  "term_id": "GO:0051601",
  "gene_symbol": "EXOC3L1",
  "gene": "UniProtKB:Q86VI1",
  "term_label": "exocyst localization",
  "gene_name": "Exocyst complex component 3-like protein"
}